L-xylulokinase activity [GO:0008744] (molecular function) Relationships: is a type of carbohydrate kinase activity [GO:0019200] Also known as: ATP:L-xylulose 5-phosphotransferase activity, L-xylulokinase (phosphorylating), L-xylulose kinase activity Definition: Catalysis of the reaction: ATP + L-xylulose = ADP + L-xylulose 5-phosphate. Sources: EC:2.7.1.53